regulation of heart rate by hormone [GO:0003064] (biological process) Also known as: hormonal cardiac chronotropy, regulation of the rate of heart contraction by hormone Relationships: is a type of regulation of heart rate by chemical signal [GO:0003062] Definition: The process in which the hormones modulates the rate of heart muscle contraction. A hormone is one of a group of substances formed in very small amounts in one specialized organ or group of cells and carried (sometimes in the bloodstream) to another organ or group of cells, in the same organism, upon which they have a specific regulatory action. Sources: GOC:mtg_cardio, GOC:rl